{
  "gene_symbol": "EIF3M",
  "gene": "UniProtKB:Q7L2H7",
  "term_label": "Unknown molecular function",
  "gene_name": "Eukaryotic translation initiation factor 3 subunit M",
  "term_id": "UNKNOWN:0001"
}